base-excision repair, gap-filling [GO:0006287] (biological process) Sources: ISBN:1550091131 Definition: Repair of the damaged strand by the combined action of an apurinic endouclease that degrades a few bases on the damaged strand and a polymerase that synthesizes a 'patch' in the 5' to 3' direction, using the undamaged strand as a template. Relationships: is a type of DNA metabolic process [GO:0006259]; is part of base-excision repair [GO:0006284]